{
  "gene": "UniProtKB:P13010",
  "gene_name": "X-ray repair cross-complementing protein 5",
  "gene_symbol": "XRCC5",
  "term_label": "double-strand break repair via nonhomologous end joining",
  "term_id": "GO:0006303"
}